{
  "gene_symbol": "CHP2",
  "term_id": "GO:0070886",
  "gene": "UniProtKB:O43745",
  "term_label": "positive regulation of calcineurin-NFAT signaling cascade",
  "gene_name": "Calcineurin B homologous protein 2"
}